GATOR1 complex binding [GO:0106080] (molecular function) Definition: Binding to a GATOR1 complex. References: PMID:28199306 Relationships: is a type of protein-containing complex binding [GO:0044877]